{
  "term_label": "serotonin biosynthetic process from tryptophan",
  "gene_symbol": "TPH1",
  "gene": "UniProtKB:P17752",
  "gene_name": "Tryptophan 5-hydroxylase 1",
  "term_id": "GO:0006587"
}